microtubule stabilizing activity [GO:0140778] (molecular function) Definition: A protein-containing complex stabilizing activity that prevents dissociation of microtubules. Relationships: is_a protein-containing complex stabilizing activity [GO:0140777] References: PMID:34970964